ribosomal small subunit export from nucleus [GO:0000056] (biological process) Definition: The directed movement of a ribosomal small subunit from the nucleus into the cytoplasm. Sources: GOC:mah Also known as: ribosomal small subunit export from cell nucleus, ribosomal small subunit export out of nucleus, ribosomal small subunit transport from nucleus to cytoplasm, ribosomal small subunit-nucleus export, 30S ribosomal subunit export from nucleus, 40S ribosomal subunit export from nucleus Relationships: is a type of GO:0000054 Regulation: regulated by regulation of ribosomal small subunit export from nucleus [GO:2000206]; negatively regulated by negative regulation of ribosomal small subunit export from nucleus [GO:2000207]; positively regulated by positive regulation of ribosomal small subunit export from nucleus [GO:2000208]